{
  "term_id": "UNKNOWN:0003",
  "gene_symbol": "MEX3A",
  "gene_name": "RNA-binding protein MEX3A",
  "gene": "UniProtKB:A1L020",
  "term_label": "Unknown cellular component"
}